{
  "gene": "UniProtKB:Q8IWV8",
  "term_label": "ubiquitin protein ligase activity",
  "gene_name": "E3 ubiquitin-protein ligase UBR2",
  "term_id": "GO:0061630",
  "gene_symbol": "UBR2"
}